{
  "term_label": "lipase activity",
  "gene_name": "Lipase member N",
  "gene_symbol": "LIPN",
  "term_id": "GO:0016298",
  "gene": "UniProtKB:Q5VXI9"
}